TRAIL-activated apoptotic signaling pathway [GO:0036462] (biological process) Definition: An extrinsic apoptotic signaling pathway initiated by the binding of the ligand TRAIL (tumor necrosis factor-related apoptosis-inducing ligand) to a death receptor on the cell surface. References: PMID:21785459 Sources: GOC:PARL, GOC:bf Also known as: TRAIL-activated extrinsic apoptotic signaling pathway, TRAIL-induced apoptotic signaling pathway, tumor necrosis factor-related apoptosis-inducing ligand apoptotic signaling pathway Regulation: regulated by regulation of TRAIL-activated apoptotic signaling pathway [GO:1903121]; negatively regulated by negative regulation of TRAIL-activated apoptotic signaling pathway [GO:1903122]; positively regulated by positive regulation of TRAIL-activated apoptotic signaling pathway [GO:1903984] Relationships: is_a extrinsic apoptotic signaling pathway via death domain receptors [GO:0008625]